{
  "gene_name": "Cadherin-related family member 2",
  "gene_symbol": "CDHR2",
  "term_label": "cell-cell adhesion mediated by cadherin",
  "gene": "UniProtKB:Q9BYE9",
  "term_id": "GO:0044331"
}